{
  "gene_symbol": "METTL21EP",
  "term_id": "UNKNOWN:0002",
  "gene_name": "Putative methyltransferase-like protein 21E pseudogene",
  "term_label": "Unknown biological process",
  "gene": "UniProtKB:A6NDL7"
}